{
  "term_label": "Unknown biological process",
  "term_id": "UNKNOWN:0002",
  "gene_name": "Uncharacterized protein C17orf107",
  "gene_symbol": "C17orf107",
  "gene": "UniProtKB:Q6ZR85"
}